{
  "term_label": "D-xylulokinase activity",
  "term_id": "GO:0004856",
  "gene_symbol": "XYLB",
  "gene_name": "Xylulose kinase",
  "gene": "UniProtKB:O75191"
}